U4 snRNA binding [GO:0030621] (molecular function) Definition: Binding to a U4 small nuclear RNA (U4 snRNA). Sources: GOC:jl Relationships: is_a GO:0017069